arciform density [GO:0098682] (cellular component) References: PMID:15626493 Relationships: is_a intracellular membraneless organelle [GO:0043232]; is part of GO:0097470 Definition: An electron dense structure that anchors a synaptic ribbon to the presynaptic membrane.